{
  "term_label": "sarcolemma",
  "term_id": "GO:0042383",
  "gene": "UniProtKB:Q13326",
  "gene_symbol": "SGCG",
  "gene_name": "Gamma-sarcoglycan"
}